{
  "gene": "UniProtKB:O75439",
  "term_id": "GO:0006627",
  "gene_name": "Mitochondrial-processing peptidase subunit beta",
  "term_label": "protein processing involved in protein targeting to mitochondrion",
  "gene_symbol": "PMPCB"
}